positive regulation of proteoglycan biosynthetic process [GO:1902730] (biological process) Subtypes: GO:0010909 Also known as: positive regulation of proteoglycan anabolism, positive regulation of proteoglycan biosynthesis, positive regulation of proteoglycan formation, positive regulation of proteoglycan synthesis, up regulation of proteoglycan anabolism, up regulation of proteoglycan biosynthesis, up regulation of proteoglycan biosynthetic process, up regulation of proteoglycan formation, up regulation of proteoglycan synthesis, up-regulation of proteoglycan anabolism, up-regulation of proteoglycan biosynthesis, up-regulation of proteoglycan biosynthetic process, up-regulation of proteoglycan formation, up-regulation of proteoglycan synthesis, upregulation of proteoglycan anabolism, upregulation of proteoglycan biosynthesis, upregulation of proteoglycan biosynthetic process, upregulation of proteoglycan formation, upregulation of proteoglycan synthesis, activation of proteoglycan anabolism, activation of proteoglycan biosynthesis, activation of proteoglycan biosynthetic process, activation of proteoglycan formation, activation of proteoglycan synthesis Definition: Any process that activates or increases the frequency, rate or extent of the chemical reactions and pathways resulting in the formation of proteoglycans, any glycoprotein in which the carbohydrate units are glycosaminoglycans. References: PMID:23212449 Sources: GOC:TermGenie, GO_REF:0000058 Relationships: is_a GO:0010560; positively regulates GO:0030166